{
  "term_id": "UNKNOWN:0002",
  "gene_name": "ADP-ribosylation factor-like protein 16",
  "gene": "UniProtKB:Q0P5N6",
  "term_label": "Unknown biological process",
  "gene_symbol": "ARL16"
}